{
  "gene_name": "Uncharacterized protein SPEM3",
  "gene": "UniProtKB:A0A1B0GUW6",
  "gene_symbol": "SPEM3",
  "term_label": "Unknown molecular function",
  "term_id": "UNKNOWN:0001"
}